{
  "gene_symbol": "ARPC5L",
  "term_label": "Arp2/3 protein complex",
  "term_id": "GO:0005885",
  "gene": "UniProtKB:Q9BPX5",
  "gene_name": "Actin-related protein 2_3 complex subunit 5-like protein"
}